{
  "term_label": "regulation of transcription by RNA polymerase II",
  "gene_name": "Zinc finger protein 182",
  "gene_symbol": "ZNF182",
  "gene": "UniProtKB:P17025",
  "term_id": "GO:0006357"
}